{
  "term_id": "GO:0002227",
  "term_label": "innate immune response in mucosa",
  "gene_name": "Histone H2B type 1-M",
  "gene_symbol": "H2BC14",
  "gene": "UniProtKB:Q99879"
}